{
  "gene_symbol": "NUDT4B",
  "gene_name": "Diphosphoinositol polyphosphate phosphohydrolase NUDT4B",
  "term_id": "GO:0034432",
  "term_label": "bis(5'-adenosyl)-pentaphosphatase activity",
  "gene": "UniProtKB:A0A024RBG1"
}